{
  "gene_name": "Melanocyte-stimulating hormone receptor",
  "term_id": "GO:0141163",
  "term_label": "positive regulation of cAMP/PKA signal transduction",
  "gene_symbol": "MC1R",
  "gene": "UniProtKB:Q01726"
}